oocyte nucleus migration involved in oocyte dorsal/ventral axis specification [GO:0007312] (BP) Sources: GOC:dph, GOC:mah, GOC:mtg_sensu, GOC:tb Definition: The directed movement of the oocyte nucleus within the cell as part of the establishment and maintenance of the dorsal/ventral axis of the oocyte. An example of this is found in Drosophila melanogaster. Relationships: is a type of nuclear migration [GO:0007097]; is a type of oocyte nucleus localization involved in oocyte dorsal/ventral axis specification [GO:0051663] Also known as: establishment of localization of oocyte nucleus during oocyte axis determination, establishment of oocyte nucleus localization during oocyte axis determination, nucleus positioning in oocyte during oocyte axis determination, oocyte axis determination, establishment of localization of nucleus, oocyte axis determination, establishment of oocyte nucleus localization, oocyte axis determination, establishment of position of nucleus, oocyte axis determination, positioning of nucleus, oocyte nucleus positioning during oocyte axis determination, oocyte axis determination, oocyte nuclear migration, oocyte axis determination, oocyte nucleus migration, oocyte nuclear migration during oocyte axis determination, oocyte nucleus migration during oocyte axis determination, establishment of oocyte nucleus localisation involved in oocyte dorsal/ventral axis specification, establishment of oocyte nucleus localization involved in oocyte dorsal-ventral axis specification, establishment of oocyte nucleus localization involved in oocyte dorsal/ventral axis determination, establishment of oocyte nucleus localization involved in oocyte dorsal/ventral axis specification, establishment of oocyte nucleus localization involved in oocyte dorsoventral axis specification, oocyte nucleus migration during oocyte axis specification